{
  "gene_symbol": "RABL6",
  "term_label": "nucleus",
  "gene_name": "Rab-like protein 6",
  "term_id": "GO:0005634",
  "gene": "UniProtKB:Q3YEC7"
}